{
  "term_id": "GO:0005737",
  "gene_symbol": "TRIM49C",
  "term_label": "cytoplasm",
  "gene_name": "Tripartite motif-containing protein 49C",
  "gene": "UniProtKB:P0CI26"
}